inositol 5-diphosphate pentakisphosphate 5-kinase activity [GO:0052836] (molecular function) Relationships: is a type of phosphotransferase activity, alcohol group as acceptor [GO:0016773]; is a type of inositol phosphate kinase activity [GO:0180030] References: PMID:11502751, PMID:18355727 Definition: Catalysis of the reaction: ATP + 5-diphospho-1D-myo-inositol pentakisphosphate = ADP + 5-triphospho-1D-myo-inositol pentakisphosphate.